{
  "gene_name": "Popeye domain-containing protein 3",
  "gene_symbol": "POPDC3",
  "term_label": "heart development",
  "gene": "UniProtKB:Q9HBV1",
  "term_id": "GO:0007507"
}